{
  "gene_name": "Ras-associating and dilute domain-containing protein",
  "term_label": "microtubule",
  "term_id": "GO:0005874",
  "gene": "UniProtKB:Q96JH8",
  "gene_symbol": "RADIL"
}